{
  "gene_symbol": "SUPV3L1",
  "term_label": "mitochondrial RNA 3'-end processing",
  "gene": "UniProtKB:Q8IYB8",
  "term_id": "GO:0000965",
  "gene_name": "ATP-dependent RNA helicase SUPV3L1, mitochondrial"
}